{
  "gene_symbol": "CHTF18",
  "gene": "UniProtKB:Q8WVB6",
  "term_label": "DNA binding",
  "term_id": "GO:0003677",
  "gene_name": "Chromosome transmission fidelity protein 18 homolog"
}